{
  "term_label": "cilium assembly",
  "term_id": "GO:0060271",
  "gene_name": "EH domain-containing protein 3",
  "gene": "UniProtKB:Q9NZN3",
  "gene_symbol": "EHD3"
}